{
  "term_id": "GO:0098882",
  "gene_symbol": "RIMS3",
  "gene": "UniProtKB:Q9UJD0",
  "gene_name": "Regulating synaptic membrane exocytosis protein 3",
  "term_label": "structural constituent of presynaptic active zone"
}